{
  "gene_name": "Melanotransferrin",
  "gene": "UniProtKB:P08582",
  "term_label": "recycling endosome",
  "term_id": "GO:0055037",
  "gene_symbol": "MELTF"
}